{
  "gene": "UniProtKB:Q7Z2R9",
  "term_id": "UNKNOWN:0002",
  "term_label": "Unknown biological process",
  "gene_symbol": "SSBP3-AS1",
  "gene_name": "Putative uncharacterized protein SSBP3-AS1"
}